{
  "gene_symbol": "CNTF",
  "gene": "UniProtKB:P26441",
  "gene_name": "Ciliary neurotrophic factor",
  "term_id": "GO:0070120",
  "term_label": "ciliary neurotrophic factor-mediated signaling pathway"
}